{
  "gene_symbol": "AGBL2",
  "term_id": "GO:0005737",
  "gene_name": "Cytosolic carboxypeptidase 2",
  "gene": "UniProtKB:Q5U5Z8",
  "term_label": "cytoplasm"
}